{
  "term_id": "GO:0003924",
  "gene": "UniProtKB:P19087",
  "gene_name": "Guanine nucleotide-binding protein G(t) subunit alpha-2",
  "term_label": "GTPase activity",
  "gene_symbol": "GNAT2"
}